negative regulation of protein autoubiquitination [GO:1905524] (BP) References: PMID:17237821 Sources: GOC:PARL, GOC:TermGenie, GOC:bc, GO_REF:0000058 Definition: Any process that stops, prevents or reduces the frequency, rate or extent of protein autoubiquitination. Relationships: is a type of negative regulation of protein ubiquitination [GO:0031397]; is a type of regulation of protein autoubiquitination [GO:1902498]; negatively regulates GO:0051865 Also known as: down regulation of protein auto-ubiquitination, down regulation of protein auto-ubiquitinylation, down regulation of protein autoubiquitination, down regulation of protein autoubiquitinylation, down regulation of protein self-ubiquitination, down regulation of protein self-ubiquitinylation, down-regulation of protein auto-ubiquitination, down-regulation of protein auto-ubiquitinylation, down-regulation of protein autoubiquitination, down-regulation of protein autoubiquitinylation, down-regulation of protein self-ubiquitination, down-regulation of protein self-ubiquitinylation, downregulation of protein auto-ubiquitination, downregulation of protein auto-ubiquitinylation, downregulation of protein autoubiquitination, downregulation of protein autoubiquitinylation, downregulation of protein self-ubiquitination, downregulation of protein self-ubiquitinylation, negative regulation of protein auto-ubiquitination, negative regulation of protein auto-ubiquitinylation, negative regulation of protein autoubiquitinylation, negative regulation of protein self-ubiquitination, negative regulation of protein self-ubiquitinylation, inhibition of protein auto-ubiquitination, inhibition of protein auto-ubiquitinylation, inhibition of protein autoubiquitination, inhibition of protein autoubiquitinylation, inhibition of protein self-ubiquitination, inhibition of protein self-ubiquitinylation